{
  "term_id": "GO:0005737",
  "term_label": "cytoplasm",
  "gene_name": "PRAME family member 10",
  "gene": "UniProtKB:O60809",
  "gene_symbol": "PRAMEF10"
}